phosphatidylinositol-4,5-bisphosphate 4-phosphatase activity [GO:0034597] (molecular function) Definition: Catalysis of the reaction: 1-phosphatidyl-1D-myo-inositol 4,5-bisphosphate + H2O = 1-phosphatidyl-1D-myo-inositol 3-phosphate + phosphate. Sources: GOC:mah, RHEA:25674 Also known as: 1-phosphatidyl-1D-myo-inositol-4,5-bisphosphate 4-phosphohydrolase activity, phosphatidyl-myo-inositol-4,5-bisphosphate 4-phosphohydrolase activity Relationships: is a type of phosphatidylinositol phosphate 4-phosphatase activity [GO:0034596]; is a type of phosphatidylinositol-4,5-bisphosphate phosphatase activity [GO:0106019]